aldehyde dehydrogenase (NADP+) activity [GO:0033721] (molecular function) Relationships: is a type of aldehyde dehydrogenase [NAD(P)+] activity [GO:0004030] Definition: Catalysis of the reaction: an aldehyde + NADP+ + H2O = an acid + NADPH + H+. Subtypes: GO:0018477, GO:0043796, 2-oxoaldehyde dehydrogenase (NADP+) activity [GO:0047552], aryl-aldehyde dehydrogenase (NADP+) activity [GO:0047683], acetaldehyde dehydrogenase (NADP+) activity [GO:0140088] Also known as: NADP-acetaldehyde dehydrogenase activity, NADP-dependent aldehyde dehydrogenase activity, aldehyde:NADP+ oxidoreductase activity Sources: RHEA:11888